{
  "gene_name": "Putative pro-MCH-like protein 2",
  "gene_symbol": "PMCHL2",
  "gene": "UniProtKB:Q9BQD1",
  "term_label": "Unknown cellular component",
  "term_id": "UNKNOWN:0003"
}